{
  "term_id": "GO:0005789",
  "gene_name": "ERO1-like protein beta",
  "term_label": "endoplasmic reticulum membrane",
  "gene": "UniProtKB:Q86YB8",
  "gene_symbol": "ERO1B"
}